{
  "gene": "UniProtKB:O00232",
  "term_id": "GO:0008541",
  "gene_symbol": "PSMD12",
  "term_label": "proteasome regulatory particle, lid subcomplex",
  "gene_name": "26S proteasome non-ATPase regulatory subunit 12"
}